{
  "term_label": "centriole",
  "gene_name": "Protein TALPID3",
  "gene_symbol": "KIAA0586",
  "gene": "UniProtKB:Q9BVV6",
  "term_id": "GO:0005814"
}